{
  "gene_symbol": "OAS2",
  "term_label": "negative regulation of viral genome replication",
  "gene": "UniProtKB:P29728",
  "term_id": "GO:0045071",
  "gene_name": "2'-5'-oligoadenylate synthase 2"
}